{
  "term_label": "Unknown molecular function",
  "gene_name": "Lysozyme-like protein 4",
  "gene_symbol": "LYZL4",
  "term_id": "UNKNOWN:0001",
  "gene": "UniProtKB:Q96KX0"
}